intracellularly calcium-gated channel activity [GO:0141147] (molecular function) Relationships: is a type of ligand-gated channel activity [GO:0022834] Definition: Enables the transmembrane transfer of a solute by a channel that opens when calcium ions bind on the intracellular side of the channel complex or one of its constituent parts. Subtypes: intracellularly calcium-gated chloride channel activity [GO:0005229] References: PMID:20929730, PMID:23021213